clearance of foreign intracellular RNA [GO:0099047] (biological process) Sources: GO:dos Relationships: is a type of clearance of foreign intracellular nucleic acids [GO:0099046] Definition: A defense process that protects an organism from invading foreign RNA.